radial growth involved in right ventricle morphogenesis [GO:0003244] (biological process) Definition: The morphogenic growth in which the right ventricle grows along a radial axis. Sources: GOC:mtg_heart Relationships: is a type of growth involved in heart morphogenesis [GO:0003241]; is part of cardiac right ventricle morphogenesis [GO:0003215]